{
  "gene_symbol": "IL7R",
  "gene": "UniProtKB:P16871",
  "term_id": "GO:0030097",
  "term_label": "hemopoiesis",
  "gene_name": "Interleukin-7 receptor subunit alpha"
}